{
  "gene_symbol": "EPB41L5",
  "term_id": "UNKNOWN:0001",
  "gene_name": "Band 4.1-like protein 5",
  "term_label": "Unknown molecular function",
  "gene": "UniProtKB:Q9HCM4"
}